sarcosine reductase activity [GO:0033794] (molecular function) Definition: Catalysis of the reaction: acetyl phosphate + methylamine + thioredoxin disulfide = N-methylglycine + phosphate + thioredoxin. Also known as: acetyl-phosphate methylamine:thioredoxin disulfide oxidoreductase (N-methylglycine-forming) activity Sources: EC:1.21.4.3 Relationships: is a type of GO:0050485